{
  "term_id": "GO:1901255",
  "gene_name": "DNA repair protein complementing XP-A cells",
  "gene_symbol": "XPA",
  "gene": "UniProtKB:P23025",
  "term_label": "nucleotide-excision repair involved in interstrand cross-link repair"
}